glycogen catabolic process via dextrin and maltose [GO:0160252] (biological process) Sources: MetaCyc:GLYCOCAT-PWY Definition: The chemical reactions and pathways resulting in the breakdown of glycogen, a polydisperse, highly branched glucan composed of chains of D-glucose residues, occurring through dextrin and maltose derivative intermediates. Relationships: is_a glycogen catabolic process [GO:0005980]